antigen processing and presentation of exogenous peptide antigen via MHC class I, TAP-independent [GO:0002480] (biological process) Relationships: is a type of antigen processing and presentation of exogenous peptide antigen via MHC class I [GO:0042590] Definition: The process in which an antigen-presenting cell expresses a peptide antigen of exogenous origin on its cell surface in association with an MHC class I protein complex following intracellular transport via a pathway not requiring TAP (transporter associated with antigen processing). The peptide is typically a fragment of a larger exogenous protein which has been degraded within the cell. Class I here refers to classical class I molecules. Also known as: cross presentation, cross-presentation, TAP-independent antigen processing and presentation of exogenous peptide antigen via MHC class I, TAP-independent exogenous peptide antigen processing and presentation via MHC class I, exogenous peptide antigen processing and presentation via MHC class I, TAP-independent References: PMID:15224093, PMID:15771591, PMID:16181335 Sources: GOC:add